{
  "term_label": "Unknown cellular component",
  "gene_symbol": "DUT",
  "term_id": "UNKNOWN:0003",
  "gene": "UniProtKB:P33316",
  "gene_name": "Deoxyuridine 5'-triphosphate nucleotidohydrolase, mitochondrial"
}